neuromedin K receptor activity [GO:0016498] (molecular function) Definition: Combining with neuromedin K, the peptide Asp-Met-His-Asp-Phe-Phe-Val-Gly-Leu-Met to initiate a change in cell activity. Relationships: is a type of tachykinin receptor activity [GO:0004995] Sources: GOC:mah, ISBN:0198506732 Also known as: neurokinin B receptor activity